{
  "gene": "UniProtKB:Q9H222",
  "term_id": "GO:0043190",
  "gene_name": "ATP-binding cassette sub-family G member 5",
  "term_label": "ATP-binding cassette (ABC) transporter complex",
  "gene_symbol": "ABCG5"
}